{
  "term_label": "cell migration",
  "gene": "UniProtKB:Q03167",
  "term_id": "GO:0016477",
  "gene_symbol": "TGFBR3",
  "gene_name": "Transforming growth factor beta receptor type 3"
}